{
  "term_label": "Unknown molecular function",
  "gene": "UniProtKB:P52943",
  "gene_name": "Cysteine-rich protein 2",
  "term_id": "UNKNOWN:0001",
  "gene_symbol": "CRIP2"
}